protein deneddylation [GO:0000338] (biological process) Regulation: regulated by regulation of protein deneddylation [GO:0060625] Sources: GOC:krc Also known as: cullin deneddylation Relationships: is a type of protein modification by small protein removal [GO:0070646] Definition: The removal of a ubiquitin-like protein of the NEDD8 type from a protein.